{
  "gene": "UniProtKB:O43316",
  "term_id": "GO:0000981",
  "gene_symbol": "PAX4",
  "gene_name": "Paired box protein Pax-4",
  "term_label": "DNA-binding transcription factor activity, RNA polymerase II-specific"
}